{
  "gene_symbol": "NELFCD",
  "gene": "UniProtKB:Q8IXH7",
  "term_label": "NELF complex",
  "term_id": "GO:0032021",
  "gene_name": "Negative elongation factor C_D"
}